{
  "gene_name": "Glucoside xylosyltransferase 2",
  "gene": "UniProtKB:A0PJZ3",
  "gene_symbol": "GXYLT2",
  "term_label": "UDP-xylosyltransferase activity",
  "term_id": "GO:0035252"
}